{
  "gene_name": "Transmembrane emp24 domain-containing protein 5",
  "term_id": "GO:0005794",
  "gene_symbol": "TMED5",
  "term_label": "Golgi apparatus",
  "gene": "UniProtKB:Q9Y3A6"
}